{
  "term_label": "somatic hypermutation of immunoglobulin genes",
  "term_id": "GO:0016446",
  "gene": "UniProtKB:P54278",
  "gene_name": "Mismatch repair endonuclease PMS2",
  "gene_symbol": "PMS2"
}